{
  "gene": "UniProtKB:O60662",
  "term_label": "regulation of myoblast proliferation",
  "gene_name": "Kelch-like protein 41",
  "gene_symbol": "KLHL41",
  "term_id": "GO:2000291"
}